{
  "term_label": "negative regulation of canonical NF-kappaB signal transduction",
  "gene_symbol": "NLRC3",
  "gene_name": "NLR family CARD domain-containing protein 3",
  "gene": "UniProtKB:Q7RTR2",
  "term_id": "GO:0043124"
}